inositol-1,4,5-trisphosphate 6-kinase activity [GO:0000823] (molecular function) Also known as: IpmK, inositol polyphosphate multikinase activity, inositol trisphosphate 6-kinase activity Sources: RHEA:17717 Relationships: is a type of inositol trisphosphate kinase activity [GO:0051766] Definition: Catalysis of the reaction: 1D-myo-inositol 1,4,5-trisphosphate + ATP = 1D-myo-inositol 1,4,5,6-tetrakisphosphate + ADP + H+.